{
  "term_id": "GO:0004674",
  "gene_name": "Serine_threonine-protein kinase Nek2",
  "gene_symbol": "NEK2",
  "term_label": "protein serine/threonine kinase activity",
  "gene": "UniProtKB:P51955"
}